{
  "term_id": "GO:0005615",
  "term_label": "extracellular space",
  "gene": "UniProtKB:O75556",
  "gene_name": "Mammaglobin-B",
  "gene_symbol": "SCGB2A1"
}